{
  "gene_name": "Arf-GAP domain and FG repeat-containing protein 2",
  "gene_symbol": "AGFG2",
  "term_id": "GO:0045109",
  "gene": "UniProtKB:O95081",
  "term_label": "intermediate filament organization"
}